{
  "gene_symbol": "GPR183",
  "term_label": "Unknown cellular component",
  "gene": "UniProtKB:P32249",
  "term_id": "UNKNOWN:0003",
  "gene_name": "G-protein coupled receptor 183"
}